{
  "term_id": "GO:0008017",
  "gene_name": "Girdin",
  "term_label": "microtubule binding",
  "gene": "UniProtKB:Q3V6T2",
  "gene_symbol": "CCDC88A"
}